growth hormone activity [GO:0070186] (molecular function) References: PMID:11445442 Sources: GOC:BHF, GOC:mah Relationships: is a type of hormone activity [GO:0005179] Also known as: GH activity, pituitary growth hormone activity, placental growth hormone activity Definition: The action characteristic of growth hormone, a peptide hormone that is secreted by the anterior pituitary or the placenta into the circulation, and binds to membrane receptors in target tissues to stimulate body growth.